{
  "gene": "UniProtKB:O15078",
  "term_id": "GO:0043010",
  "term_label": "camera-type eye development",
  "gene_name": "Centrosomal protein of 290 kDa",
  "gene_symbol": "CEP290"
}